{
  "gene_symbol": "SLC35B2",
  "term_label": "3'-phosphoadenosine 5'-phosphosulfate transport",
  "gene": "UniProtKB:Q8TB61",
  "gene_name": "Adenosine 3'-phospho 5'-phosphosulfate transporter 1",
  "term_id": "GO:0046963"
}